{
  "gene": "UniProtKB:Q969K3",
  "term_label": "plasma membrane",
  "gene_name": "E3 ubiquitin-protein ligase RNF34",
  "term_id": "GO:0005886",
  "gene_symbol": "RNF34"
}